{
  "gene_name": "Killer cell lectin-like receptor subfamily F member 2",
  "gene": "UniProtKB:D3W0D1",
  "term_label": "Unknown biological process",
  "gene_symbol": "KLRF2",
  "term_id": "UNKNOWN:0002"
}